nuclear receptor-mediated signaling pathway [GO:0141193] (biological process) References: PMID:25614732 Definition: The series of molecular signals initiated by a signaling molecule binding to an intracellular receptor of the nuclear receptor protein family, and ending with regulation of a downstream cellular process, e.g. transcription. Subtypes: GO:0002154, GO:0030518, GO:0035357, nuclear receptor-mediated bile acid signaling pathway [GO:0038185], retinoic acid receptor signaling pathway [GO:0048384], GO:0070561 Also known as: nuclear receptor signaling pathway Relationships: is a type of intracellular receptor signaling pathway [GO:0030522]